2-dehydro-3-deoxy-D-pentonate aldolase activity [GO:0047440] (MF) Definition: Catalysis of the reaction: 2-dehydro-3-deoxy-D-arabinonate = glycolaldehyde + pyruvate. Sources: EC:4.1.2.28, RHEA:20609 Relationships: is a type of GO:0016832 Also known as: 3-deoxy-D-pentulosonic acid aldolase, 2-dehydro-3-deoxy-D-pentonate glycolaldehyde-lyase activity, 2-keto-3-deoxy-D-pentonate aldolase activity